{
  "term_label": "Unknown biological process",
  "term_id": "UNKNOWN:0002",
  "gene": "UniProtKB:Q05315",
  "gene_name": "Galectin-10",
  "gene_symbol": "CLC"
}